MAML1-RBP-Jkappa- ICN1 complex [GO:0002193] (cellular component) References: PMID:16510869 Sources: CORUM:2949 Also known as: MAML1-CSL-ICN1, MAML1-CSL-Notch1 complex, MAML1-RBP-Jkappa-Notch1 complex Definition: A protein complex that consists of the intracellular domain of Notch1 (ICN1), the DNA-binding transcription factor RBP-Jkappa, and the transcriptional coactivator Mastermind-like-1 (MAML1); the complex is involved in transcriptional activation in response to Notch-mediated signaling. Relationships: is a type of protein-containing complex [GO:0032991]